{
  "term_label": "GTPase activator activity",
  "gene": "UniProtKB:Q66K14",
  "gene_symbol": "TBC1D9B",
  "gene_name": "TBC1 domain family member 9B",
  "term_id": "GO:0005096"
}